{
  "gene_symbol": "DNASE1L1",
  "term_id": "GO:0005634",
  "term_label": "nucleus",
  "gene": "UniProtKB:P49184",
  "gene_name": "Deoxyribonuclease-1-like 1"
}